{
  "gene_symbol": "MX1",
  "term_id": "GO:0008017",
  "gene_name": "Interferon-induced GTP-binding protein Mx1",
  "term_label": "microtubule binding",
  "gene": "UniProtKB:P20591"
}